{
  "gene_name": "PIH1 domain-containing protein 1",
  "gene_symbol": "PIH1D1",
  "term_label": "ribonucleoprotein complex",
  "gene": "UniProtKB:Q9NWS0",
  "term_id": "GO:1990904"
}